{
  "gene_symbol": "HDGFL3",
  "gene": "UniProtKB:Q9Y3E1",
  "term_label": "Unknown molecular function",
  "term_id": "UNKNOWN:0001",
  "gene_name": "Hepatoma-derived growth factor-related protein 3"
}